{
  "gene": "UniProtKB:O14513",
  "gene_name": "Nck-associated protein 5",
  "gene_symbol": "NCKAP5",
  "term_label": "microtubule bundle formation",
  "term_id": "GO:0001578"
}